{
  "gene": "UniProtKB:Q96KR6",
  "term_id": "UNKNOWN:0002",
  "gene_symbol": "FAM210B",
  "term_label": "Unknown biological process",
  "gene_name": "Protein FAM210B, mitochondrial"
}